{
  "gene_symbol": "ACTA1",
  "term_id": "GO:0005865",
  "term_label": "striated muscle thin filament",
  "gene_name": "Actin, alpha skeletal muscle",
  "gene": "UniProtKB:P68133"
}